{
  "gene_name": "Uncharacterized protein C15orf61",
  "term_id": "UNKNOWN:0003",
  "term_label": "Unknown cellular component",
  "gene": "UniProtKB:A6NNL5",
  "gene_symbol": "C15orf61"
}